{
  "term_label": "potassium ion leak channel activity",
  "gene_name": "Potassium channel subfamily K member 4",
  "term_id": "GO:0022841",
  "gene": "UniProtKB:Q9NYG8",
  "gene_symbol": "KCNK4"
}